{
  "gene": "UniProtKB:P49913",
  "term_label": "lipopolysaccharide binding",
  "term_id": "GO:0001530",
  "gene_name": "Cathelicidin antimicrobial peptide",
  "gene_symbol": "CAMP"
}